outer membrane [GO:0019867] (CC) Definition: The external membrane of Gram-negative bacteria or certain organelles such as mitochondria and chloroplasts; freely permeable to most ions and metabolites. Sources: GOC:go_curators Relationships: is a type of membrane [GO:0016020] Subtypes: cell outer membrane [GO:0009279], organelle outer membrane [GO:0031968], outer endospore membrane [GO:0043594]